regulation of adaxial/abaxial pattern formation [GO:2000011] (biological process) Also known as: regulation of adaxial/abaxial pattern specification Sources: GOC:obol Definition: Any process that modulates the frequency, rate or extent of adaxial/abaxial pattern formation. Relationships: is a type of regulation of multicellular organismal process [GO:0051239]; regulates GO:0009955